{
  "term_label": "chloride channel activity",
  "gene": "UniProtKB:Q8N1M1",
  "gene_name": "Bestrophin-3",
  "term_id": "GO:0005254",
  "gene_symbol": "BEST3"
}